{
  "gene_symbol": "GIMAP1",
  "term_label": "endoplasmic reticulum",
  "gene_name": "GTPase IMAP family member 1",
  "gene": "UniProtKB:Q8WWP7",
  "term_id": "GO:0005783"
}